{
  "gene_name": "Protein tyrosine phosphatase type IVA 1",
  "gene": "UniProtKB:Q93096",
  "term_id": "GO:0005737",
  "term_label": "cytoplasm",
  "gene_symbol": "PTP4A1"
}